{
  "gene_name": "Elongation factor 1-alpha 2",
  "term_id": "UNKNOWN:0003",
  "term_label": "Unknown cellular component",
  "gene": "UniProtKB:Q05639",
  "gene_symbol": "EEF1A2"
}